{
  "gene_name": "Calcium homeostasis modulator protein 3",
  "term_label": "monoatomic cation channel activity",
  "gene_symbol": "CALHM3",
  "term_id": "GO:0005261",
  "gene": "UniProtKB:Q86XJ0"
}